{
  "gene": "UniProtKB:Q16181",
  "term_label": "molecular adaptor activity",
  "term_id": "GO:0060090",
  "gene_name": "Septin-7",
  "gene_symbol": "SEPTIN7"
}